{
  "term_label": "central nervous system development",
  "gene_symbol": "VAX2",
  "gene": "UniProtKB:Q9UIW0",
  "term_id": "GO:0007417",
  "gene_name": "Ventral anterior homeobox 2"
}